{
  "term_id": "GO:0004735",
  "gene_symbol": "PYCR2",
  "gene_name": "Pyrroline-5-carboxylate reductase 2",
  "gene": "UniProtKB:Q96C36",
  "term_label": "pyrroline-5-carboxylate reductase activity"
}